{
  "term_id": "GO:0005886",
  "gene_name": "Killer cell lectin-like receptor subfamily F member 1",
  "term_label": "plasma membrane",
  "gene_symbol": "KLRF1",
  "gene": "UniProtKB:Q9NZS2"
}